{
  "gene_name": "Heat shock protein 75 kDa, mitochondrial",
  "term_id": "GO:0051082",
  "term_label": "unfolded protein binding",
  "gene_symbol": "TRAP1",
  "gene": "UniProtKB:Q12931"
}